{
  "term_label": "Sin3-type complex",
  "gene_name": "Paired amphipathic helix protein Sin3a",
  "term_id": "GO:0070822",
  "gene_symbol": "SIN3A",
  "gene": "UniProtKB:Q96ST3"
}